{
  "term_label": "nucleus",
  "gene_symbol": "TRIAP1",
  "term_id": "GO:0005634",
  "gene": "UniProtKB:O43715",
  "gene_name": "TP53-regulated inhibitor of apoptosis 1"
}